{
  "gene": "UniProtKB:Q9UH73",
  "term_label": "RNA polymerase II cis-regulatory region sequence-specific DNA binding",
  "gene_symbol": "EBF1",
  "term_id": "GO:0000978",
  "gene_name": "Transcription factor COE1"
}